{
  "gene_name": "Translation initiation factor eIF-2B subunit epsilon",
  "term_label": "eukaryotic translation initiation factor 2B complex",
  "gene_symbol": "EIF2B5",
  "term_id": "GO:0005851",
  "gene": "UniProtKB:Q13144"
}